{
  "term_label": "retrograde axonal transport",
  "term_id": "GO:0008090",
  "gene_name": "F-box_WD repeat-containing protein 11",
  "gene": "UniProtKB:Q9UKB1",
  "gene_symbol": "FBXW11"
}